{
  "term_id": "GO:0000149",
  "gene": "UniProtKB:Q8IV01",
  "gene_name": "Synaptotagmin-12",
  "term_label": "SNARE binding",
  "gene_symbol": "SYT12"
}